histone H2B acetyltransferase activity [GO:0044013] (molecular function) References: PMID:19056256 Definition: Catalysis of the reaction: acetyl-CoA + histone H2B L-lysine = CoA + histone H2B N6-acetyl-L-lysine. Also known as: H2B histone acetylase activity, H2B histone acetyltransferase activity, H2B histone lysine N-acetyltransferase activity Relationships: is a type of histone acetyltransferase activity [GO:0004402] Subtypes: histone H2BK5 acetyltransferase activity [GO:0044014], histone H2BK12 acetyltransferase activity [GO:0044015]